regulation of immature T cell proliferation in thymus [GO:0033084] (biological process) Definition: Any process that modulates the frequency, rate or extent of immature T cell proliferation in the thymus. Sources: GOC:add, GOC:mah Subtypes: negative regulation of immature T cell proliferation in thymus [GO:0033088], positive regulation of immature T cell proliferation in thymus [GO:0033092] Relationships: is a type of GO:0033083; regulates immature T cell proliferation in thymus [GO:0033080] Note: Note that immunologists typically use the word 'development' to refer to cells of B or T cell lineages undergoing the process that GO describes as 'cell differentiation'. Also known as: regulation of thymic T cell proliferation, regulation of thymocyte cell proliferation, regulation of thymocyte proliferation